alcohol oxidase activity [GO:0047639] (molecular function) Sources: EC:1.1.3.13, MetaCyc:ALCOHOL-OXIDASE-RXN Also known as: AOX activity, alcohol:oxygen oxidoreductase activity, ethanol oxidase activity Relationships: is a type of GO:0016899 Definition: Catalysis of the reaction: a primary alcohol + O2 = an aldehyde + H2O2.